{
  "term_id": "GO:0006886",
  "gene_name": "Rab-like protein 2B",
  "gene": "UniProtKB:Q9UNT1",
  "gene_symbol": "RABL2B",
  "term_label": "intracellular protein transport"
}